lambdoid suture morphogenesis [GO:0060366] (biological process) Definition: The process in which the lambdoid suture is generated and organized. Sources: GOC:dph, GOC:sl Relationships: is a type of cranial suture morphogenesis [GO:0060363]